{
  "gene": "UniProtKB:O95825",
  "term_label": "Unknown cellular component",
  "gene_symbol": "CRYZL1",
  "term_id": "UNKNOWN:0003",
  "gene_name": "Quinone oxidoreductase-like protein 1"
}